{
  "gene_name": "WD repeat-containing protein 19",
  "gene": "UniProtKB:Q8NEZ3",
  "gene_symbol": "WDR19",
  "term_label": "intraciliary retrograde transport",
  "term_id": "GO:0035721"
}